{
  "term_id": "GO:2000234",
  "gene": "UniProtKB:Q9UI30",
  "term_label": "positive regulation of rRNA processing",
  "gene_name": "Multifunctional methyltransferase subunit TRM112-like protein",
  "gene_symbol": "TRMT112"
}